{
  "gene": "UniProtKB:Q9Y603",
  "gene_name": "Transcription factor ETV7",
  "term_label": "cell differentiation",
  "gene_symbol": "ETV7",
  "term_id": "GO:0030154"
}